programmed DNA elimination [GO:0031049] (biological process) Subtypes: programmed DNA elimination by chromosome breakage [GO:0031052], programmed DNA elimination by elimination of internal DNA segments [GO:0140763] Definition: A process in which genomic fragments or entire chromosomes are eliminated from somatic cells or from micronuclei of ciliates. This process occurs in the developing macronucleus (anlage) of a ciliate, as well as in other species, including vertebrates and is an irreversible mechanism of gene silencing. References: PMID:18708581, PMID:24886889, PMID:32986476 Sources: GOC:mah, GOC:ns Relationships: is a type of negative regulation of gene expression [GO:0010629]